{
  "gene": "UniProtKB:P35523",
  "gene_symbol": "CLCN1",
  "term_id": "GO:0006821",
  "gene_name": "Chloride channel protein 1",
  "term_label": "chloride transport"
}